L-xylose 1-dehydrogenase activity [GO:0050037] (molecular function) Also known as: L-xylose dehydrogenase activity, L-xylose:NADP+ 1-oxidoreductase activity, NADPH-xylose reductase activity Sources: RHEA:15789 Relationships: is a type of oxidoreductase activity, acting on the CH-OH group of donors, NAD or NADP as acceptor [GO:0016616] Definition: Catalysis of the reaction: L-xylose + NADP+ = H+ + L-xylono-1,4-lactone + NADPH.